{
  "term_id": "UNKNOWN:0003",
  "gene_symbol": "HSD11B2",
  "term_label": "Unknown cellular component",
  "gene": "UniProtKB:P80365",
  "gene_name": "11-beta-hydroxysteroid dehydrogenase type 2"
}